{
  "gene_symbol": "HNRNPCL3",
  "gene": "UniProtKB:B7ZW38",
  "gene_name": "Heterogeneous nuclear ribonucleoprotein C-like 3",
  "term_id": "GO:0003723",
  "term_label": "RNA binding"
}